butyrate biosynthetic process [GO:0046358] (biological process) Relationships: is a type of GO:0019605; is a type of short-chain fatty acid biosynthetic process [GO:0051790] Definition: The chemical reactions and pathways resulting in the formation of butyrate, the anion of butyric acid. Subtypes: butyryl-CoA catabolic process to butyrate [GO:0044581] Also known as: butanoic acid anabolism, butanoic acid biosynthesis, butanoic acid biosynthetic process, butanoic acid formation, butanoic acid synthesis, butyrate anabolism, butyrate biosynthesis, butyrate formation, butyrate synthesis Sources: ISBN:0198506732